{
  "gene_name": "Olfactory receptor 2A1_2A42",
  "gene": "UniProtKB:Q8NGT9",
  "term_label": "detection of chemical stimulus involved in sensory perception of smell",
  "gene_symbol": "OR2A1",
  "term_id": "GO:0050911"
}